distal tip cell migration [GO:0097628] (biological process) Definition: The orderly movement of a distal tip cell. References: PMID:24968003 Sources: CL:0000661, GOC:mm2 Relationships: is a type of GO:0016477 Regulation: regulated by regulation of distal tip cell migration [GO:1903354]; negatively regulated by negative regulation of distal tip cell migration [GO:1903355]; positively regulated by GO:1903356